{
  "term_id": "GO:0005604",
  "gene_name": "Laminin subunit alpha-2",
  "gene": "UniProtKB:P24043",
  "term_label": "basement membrane",
  "gene_symbol": "LAMA2"
}